2-acylglycerol O-acyltransferase activity [GO:0003846] (molecular function) Relationships: is a type of acylglycerol O-acyltransferase activity [GO:0016411] References: PMID:4016575 Sources: RHEA:16741 Also known as: acyl coenzyme A-monoglyceride acyltransferase activity, acyl-CoA:2-acylglycerol O-acyltransferase activity, acylglycerol palmitoyltransferase activity, monoacylglycerol acyltransferase activity, monoglyceride acyltransferase activity Definition: Catalysis of the reaction: acyl-CoA + 2-acylglycerol = CoA + diacylglycerol.